renal water homeostasis [GO:0003091] (BP) Sources: GOC:mtg_cardio Definition: Renal process involved in the maintenance of an internal steady state of water in the body. Also known as: water homeostasis by the renal system Relationships: is_a GO:0003014; is a type of multicellular organismal-level water homeostasis [GO:0050891]